positive regulation of neurogenesis [GO:0050769] (biological process) Sources: GOC:ai Definition: Any process that activates or increases the frequency, rate or extent of neurogenesis, the generation of cells within the nervous system. Also known as: up regulation of neurogenesis, up-regulation of neurogenesis, upregulation of neurogenesis, activation of neurogenesis, stimulation of neurogenesis Relationships: is_a positive regulation of cell development [GO:0010720]; is a type of GO:0050767; is a type of positive regulation of nervous system development [GO:0051962]; positively regulates neurogenesis [GO:0022008] Subtypes: positive regulation of neuroblast proliferation [GO:0002052], positive regulation of gliogenesis [GO:0014015], positive regulation of long-term neuronal synaptic plasticity [GO:0048170], positive regulation of short-term neuronal synaptic plasticity [GO:0048173], positive regulation of axonogenesis [GO:0050772], positive regulation of dendrite morphogenesis [GO:0050775]